{
  "gene": "UniProtKB:P80303",
  "gene_name": "Nucleobindin-2",
  "term_label": "endoplasmic reticulum-Golgi intermediate compartment",
  "term_id": "GO:0005793",
  "gene_symbol": "NUCB2"
}